{
  "term_id": "GO:0032263",
  "term_label": "GMP salvage",
  "gene_symbol": "HPRT1",
  "gene": "UniProtKB:P00492",
  "gene_name": "Hypoxanthine-guanine phosphoribosyltransferase"
}